{
  "term_label": "extracellular space",
  "term_id": "GO:0005615",
  "gene": "UniProtKB:P10997",
  "gene_symbol": "IAPP",
  "gene_name": "Islet amyloid polypeptide"
}